{
  "gene": "UniProtKB:P12830",
  "gene_symbol": "CDH1",
  "term_label": "cell-cell adhesion mediated by cadherin",
  "gene_name": "Cadherin-1",
  "term_id": "GO:0044331"
}